molybdopterin-synthase adenylyltransferase activity [GO:0061605] (molecular function) Definition: Catalysis of the reaction: ATP [molybdopterin-synthase sulfur-carrier protein]-Gly-Gly = diphosphate [molybdopterin-synthase sulfur-carrier protein]-Gly-Gly-AMP. References: PMID:18154309, PMID:22370186 Sources: EC:2.7.7.80, GOC:dph Relationships: is_a adenylyltransferase activity [GO:0070566]